{
  "gene_name": "Fibroblast growth factor-binding protein 1",
  "gene_symbol": "FGFBP1",
  "gene": "UniProtKB:Q14512",
  "term_id": "GO:0019838",
  "term_label": "growth factor binding"
}